{
  "gene": "UniProtKB:Q71RC2",
  "gene_name": "La-related protein 4",
  "term_label": "positive regulation of translation",
  "gene_symbol": "LARP4",
  "term_id": "GO:0045727"
}